{
  "gene_symbol": "FNDC9",
  "gene_name": "Fibronectin type III domain-containing protein 9",
  "gene": "UniProtKB:Q8TBE3",
  "term_id": "UNKNOWN:0002",
  "term_label": "Unknown biological process"
}